{
  "term_label": "protein xylosyltransferase activity",
  "gene": "UniProtKB:Q86Y38",
  "gene_symbol": "XYLT1",
  "gene_name": "Xylosyltransferase 1",
  "term_id": "GO:0030158"
}